{
  "gene_symbol": "NIPSNAP3B",
  "term_id": "GO:0005739",
  "gene": "UniProtKB:Q9BS92",
  "term_label": "mitochondrion",
  "gene_name": "Protein NipSnap homolog 3B"
}